{
  "gene_symbol": "AIFM1",
  "term_label": "NAD(P)H oxidase H2O2-forming activity",
  "term_id": "GO:0016174",
  "gene_name": "Apoptosis-inducing factor 1, mitochondrial",
  "gene": "UniProtKB:O95831"
}